{
  "term_label": "negative regulation of excitatory postsynaptic potential",
  "gene": "UniProtKB:Q86YD3",
  "gene_name": "Transmembrane protein 25",
  "term_id": "GO:0090394",
  "gene_symbol": "TMEM25"
}